{
  "term_label": "ATPase activator activity",
  "term_id": "GO:0001671",
  "gene_name": "DnaJ homolog subfamily C member 15",
  "gene": "UniProtKB:Q9Y5T4",
  "gene_symbol": "DNAJC15"
}